skin development [GO:0043588] (biological process) Sources: GOC:jl, UBERON:0002097 Also known as: animal skin development Definition: The process whose specific outcome is the progression of the skin over time, from its formation to the mature structure. The skin is the external membranous integument of an animal. In vertebrates the skin generally consists of two layers, an outer nonsensitive and nonvascular epidermis (cuticle or skarfskin) composed of cells which are constantly growing and multiplying in the deeper, and being thrown off in the superficial layers, as well as an inner vascular dermis (cutis, corium or true skin) composed mostly of connective tissue. Relationships: is a type of animal organ development [GO:0048513]